{
  "term_label": "RNA binding",
  "gene_symbol": "DHX38",
  "gene_name": "Pre-mRNA-splicing factor ATP-dependent RNA helicase PRP16",
  "term_id": "GO:0003723",
  "gene": "UniProtKB:Q92620"
}